{
  "gene_symbol": "LPA",
  "term_label": "Unknown biological process",
  "gene_name": "Apolipoprotein(a)",
  "term_id": "UNKNOWN:0002",
  "gene": "UniProtKB:P08519"
}